{
  "term_label": "cytoplasmic dynein complex",
  "term_id": "GO:0005868",
  "gene_name": "Dynein light chain Tctex-type 4",
  "gene": "UniProtKB:Q5JR98",
  "gene_symbol": "DYNLT4"
}